{
  "term_id": "GO:0006103",
  "gene_symbol": "KGD4",
  "term_label": "2-oxoglutarate metabolic process",
  "gene": "UniProtKB:P82909",
  "gene_name": "Alpha-ketoglutarate dehydrogenase component 4"
}